negative regulation of chemotaxis to arachidonate [GO:1904553] (biological process) Also known as: down regulation of chemotaxis to arachidonic acid, down-regulation of chemotaxis to arachidonic acid, downregulation of chemotaxis to arachidonic acid, negative regulation of chemotaxis to arachidonic acid, inhibition of chemotaxis to arachidonic acid References: PMID:16382163 Sources: GOC:TermGenie, GO_REF:0000058 Definition: Any process that stops, prevents or reduces the frequency, rate or extent of chemotaxis to arachidonic acid. Relationships: is_a negative regulation of chemotaxis [GO:0050922]; is a type of GO:1904552; negatively regulates chemotaxis to arachidonate [GO:0034670]